phosphoglycerol geranylgeranyltransferase activity [GO:0047294] (molecular function) Relationships: is a type of prenyltransferase activity [GO:0004659] Note: This function is involved in archaeal lipid synthesis. Also known as: (S)-3-O-geranylgeranylglyceryl phosphate synthase activity, GGGP synthase activity, GGGPS activity, geranylgeranyl diphosphate:sn-glyceryl phosphate geranylgeranyltransferase activity, geranylgeranyl-transferase activity, glycerol phosphate geranylgeranyltransferase activity Definition: Catalysis of the reaction: (2E,6E,10E)-geranylgeranyl diphosphate + sn-glycerol 1-phosphate = diphosphate + sn-3-O-(geranylgeranyl)glycerol 1-phosphate. References: PMID:12801917, PMID:17253090, PMID:8408023 Sources: RHEA:23404